{
  "gene": "UniProtKB:Q8IWB6",
  "term_id": "GO:0007094",
  "term_label": "mitotic spindle assembly checkpoint signaling",
  "gene_symbol": "TEX14",
  "gene_name": "Inactive serine_threonine-protein kinase TEX14"
}